{
  "gene_name": "Gremlin-1",
  "gene": "UniProtKB:O60565",
  "gene_symbol": "GREM1",
  "term_label": "receptor ligand activity",
  "term_id": "GO:0048018"
}